{
  "gene_symbol": "OR10G6",
  "term_label": "plasma membrane",
  "term_id": "GO:0005886",
  "gene": "UniProtKB:Q8NH81",
  "gene_name": "Olfactory receptor 10G6"
}